{
  "term_id": "GO:0000976",
  "term_label": "transcription cis-regulatory region binding",
  "gene": "UniProtKB:Q52M93",
  "gene_name": "Zinc finger protein 585B",
  "gene_symbol": "ZNF585B"
}